{
  "gene": "UniProtKB:A0A075B6I1",
  "term_id": "GO:0006955",
  "gene_name": "Immunoglobulin lambda variable 4-60",
  "term_label": "immune response",
  "gene_symbol": "IGLV4-60"
}